bone maturation [GO:0070977] (biological process) Sources: GOC:dph, GOC:mah Definition: A developmental process, independent of morphogenetic (shape) change, that is required for bone to attain its fully functional state. Relationships: is a type of animal organ maturation [GO:0048799]; is part of GO:0060348